cellular response to cisplatin [GO:0072719] (biological process) Definition: Any process that results in a change in state or activity of a cell (in terms of movement, secretion, enzyme production, gene expression, etc.) as a result of a cisplatin stimulus. Sources: GOC:mah Relationships: is a type of cellular response to chemical stimulus [GO:0070887]; is a type of GO:0072718